neuron-glial cell signaling [GO:0150099] (biological process) Also known as: neuron-glia signaling, neuron-glia signalling, neuron-glial cell signalling, neurone-glia signaling, neurone-glia signalling, neurone-glial cell signaling, neurone-glial cell signalling Relationships: is a type of GO:0007267 References: PMID:10195197, PMID:10196584, PMID:10377338, PMID:10493741, PMID:11356870, PMID:11399439, PMID:15252819, PMID:27788368 Sources: GOC:aruk, GOC:bc Definition: Cell-cell signaling that mediates the transfer of information from a neuron to a glial cell. This signaling has been shown to be mediated by various molecules released by different types of neurons, e.g. glutamate, gamma-amino butyric acid (GABA), noradrenaline, acetylcholine, dopamine and adenosine.